{
  "gene": "UniProtKB:Q56UQ5",
  "gene_symbol": "Q56UQ5",
  "gene_name": "TPT1-like protein",
  "term_label": "Unknown biological process",
  "term_id": "UNKNOWN:0002"
}